{
  "gene_name": "Cytoskeleton-associated protein 5",
  "gene": "UniProtKB:Q14008",
  "gene_symbol": "CKAP5",
  "term_label": "centrosome duplication",
  "term_id": "GO:0051298"
}